{
  "gene_symbol": "SPATA6",
  "term_id": "GO:0044458",
  "gene_name": "Spermatogenesis-associated protein 6",
  "gene": "UniProtKB:Q9NWH7",
  "term_label": "motile cilium assembly"
}